fibrinogen binding [GO:0070051] (molecular function) Relationships: is a type of protein-containing complex binding [GO:0044877] Sources: GOC:BHF, GOC:mah, GOC:vk Definition: Binding to fibrinogen, a highly soluble hexameric glycoprotein complex that is found in blood plasma and is converted to fibrin by thrombin in the coagulation cascade.